interleukin-20 receptor binding [GO:0045517] (molecular function) Relationships: is a type of GO:0005126 Definition: Binding to an interleukin-20 receptor. Also known as: IL-20, interleukin-20 receptor ligand Sources: GOC:go_curators